regulation of protein localization to endoplasmic reticulum [GO:1905550] (biological process) Definition: Any process that modulates the frequency, rate or extent of protein localization to endoplasmic reticulum. References: PMID:22768340 Sources: GOC:TermGenie, GO_REF:0000058 Subtypes: negative regulation of protein localization to endoplasmic reticulum [GO:1905551], positive regulation of protein localization to endoplasmic reticulum [GO:1905552] Also known as: regulation of protein localisation in endoplasmic reticulum, regulation of protein localization in ER, regulation of protein localization in endoplasmic reticulum Relationships: is a type of regulation of protein localization [GO:0032880]; regulates protein localization to endoplasmic reticulum [GO:0070972]